2-coumarate O-beta-glucosyltransferase activity [GO:0047212] (molecular function) Sources: EC:2.4.1.114, RHEA:10236 Also known as: UDP-glucose:trans-2-hydroxycinnamate O-beta-D-glucosyltransferase activity, UDPG:o-coumaric acid O-glucosyltransferase activity, UDPglucose:trans-2-hydroxycinnamate O-beta-D-glucosyltransferase activity, uridine diphosphoglucose-o-coumarate glucosyltransferase activity Relationships: is a type of UDP-glucosyltransferase activity [GO:0035251] Definition: Catalysis of the reaction: trans-2-coumarate + UDP-D-glucose = trans-beta-D-glucosyl-2-hydroxycinnamate + H+ + UDP.